{
  "term_id": "GO:0071380",
  "term_label": "cellular response to prostaglandin E stimulus",
  "gene_symbol": "PTGER2",
  "gene": "UniProtKB:P43116",
  "gene_name": "Prostaglandin E2 receptor EP2 subtype"
}